{
  "gene": "UniProtKB:Q16663",
  "term_id": "GO:0070098",
  "gene_name": "C-C motif chemokine 15",
  "gene_symbol": "CCL15",
  "term_label": "chemokine-mediated signaling pathway"
}